ornithine decarboxylase activator activity [GO:0042978] (molecular function) Relationships: is a type of enzyme activator activity [GO:0008047]; is a type of ornithine decarboxylase regulator activity [GO:0042979]; positively regulates GO:0004586 Definition: Binds to and increases ornithine decarboxylase activity. Sources: GOC:jl Also known as: L-ornithine carboxy-lyase activator activity